{
  "term_id": "GO:0048812",
  "term_label": "neuron projection morphogenesis",
  "gene": "UniProtKB:Q9BY11",
  "gene_symbol": "PACSIN1",
  "gene_name": "Protein kinase C and casein kinase substrate in neurons protein 1"
}